{
  "gene": "UniProtKB:Q9Y3E0",
  "term_label": "membrane",
  "gene_name": "Vesicle transport protein GOT1B",
  "gene_symbol": "GOLT1B",
  "term_id": "GO:0016020"
}